{
  "gene_symbol": "IFNA8",
  "term_label": "B cell activation involved in immune response",
  "gene_name": "Interferon alpha-8",
  "term_id": "GO:0002312",
  "gene": "UniProtKB:P32881"
}